{
  "term_id": "GO:0005102",
  "gene_name": "HERV-H LTR-associating protein 2",
  "term_label": "signaling receptor binding",
  "gene_symbol": "HHLA2",
  "gene": "UniProtKB:Q9UM44"
}